cellular response to external stimulus [GO:0071496] (biological process) Definition: Any process that results in a change in state or activity of a cell (in terms of movement, secretion, enzyme production, gene expression, etc.) as a result of an external stimulus. Sources: GOC:mah Note: Note that this term is in the subset of terms that should not be used for direct gene product annotation. Instead, select a child term or, if no appropriate child term exists, please request a new term. Direct annotations to this term may be amended during annotation QC. Relationships: is a type of response to external stimulus [GO:0009605] Subtypes: cellular response to external biotic stimulus [GO:0071217], cellular response to mechanical stimulus [GO:0071260]